{
  "term_label": "zinc ion transmembrane transport",
  "gene": "UniProtKB:Q9Y6M5",
  "gene_symbol": "SLC30A1",
  "gene_name": "Proton-coupled zinc antiporter SLC30A1",
  "term_id": "GO:0071577"
}